{
  "gene": "UniProtKB:Q9UBX7",
  "term_label": "protein maturation",
  "term_id": "GO:0051604",
  "gene_name": "Kallikrein-11",
  "gene_symbol": "KLK11"
}